regulation of myosin II filament disassembly [GO:0043521] (biological process) Relationships: is a type of regulation of protein-containing complex disassembly [GO:0043244]; is a type of GO:0043519; regulates myosin II filament disassembly [GO:0031037] Definition: Any process that modulates the frequency, rate or extent of the disassembly of a bipolar filament composed of myosin II molecules. Sources: GOC:jl